{
  "term_label": "extracellular space",
  "gene": "UniProtKB:Q9GZX6",
  "gene_name": "Interleukin-22",
  "term_id": "GO:0005615",
  "gene_symbol": "IL22"
}